{
  "term_id": "GO:0005794",
  "gene_symbol": "PXYLP1",
  "gene": "UniProtKB:Q8TE99",
  "term_label": "Golgi apparatus",
  "gene_name": "2-phosphoxylose phosphatase 1"
}